{
  "gene": "UniProtKB:A0A1W2PQL4",
  "gene_name": "Zinc finger protein 722",
  "term_id": "UNKNOWN:0003",
  "term_label": "Unknown cellular component",
  "gene_symbol": "ZNF722"
}